seminal vesicle morphogenesis [GO:0061682] (biological process) Sources: GOC:dph Relationships: is a type of gland morphogenesis [GO:0022612]; is part of seminal vesicle development [GO:0061107] Definition: The process in which the anatomical structures of a seminal vesicle are generated and organized.